CTP salvage [GO:0044211] (biological process) Relationships: is_a CTP biosynthetic process [GO:0006241]; is a type of pyrimidine ribonucleotide salvage [GO:0010138] References: PMID:10501935 Sources: GOC:ecd, GOC:jl Definition: Any process which produces cytidine 5'-triphosphate (CTP) from derivatives of it, without de novo synthesis. Also known as: CTP biosynthetic process via salvage pathway, cytidine 5'-triphosphate salvage